{
  "term_label": "calcium ion binding",
  "gene_symbol": "S100B",
  "term_id": "GO:0005509",
  "gene": "UniProtKB:P04271",
  "gene_name": "Protein S100-B"
}